mitochondrion organization [GO:0007005] (biological process) Subtypes: mitochondrial fission [GO:0000266], mitochondrial membrane organization [GO:0007006], mitochondrial fusion [GO:0008053], apoptotic mitochondrial changes [GO:0008637], sperm mitochondrion organization [GO:0030382], mitochondrial respirasome assembly [GO:0097250] Also known as: mitochondria organization, mitochondrial biogenesis, mitochondrial organization, mitochondrion biogenesis, mitochondrion organisation, mitochondrion morphogenesis, mitochondrion organization and biogenesis Definition: A process that is carried out at the cellular level which results in the assembly, arrangement of constituent parts, or disassembly of a mitochondrion; includes mitochondrial morphogenesis and distribution, and replication of the mitochondrial genome as well as synthesis of new mitochondrial components. Regulation: regulated by regulation of mitochondrion organization [GO:0010821]; positively regulated by GO:1901860 Relationships: is a type of organelle organization [GO:0006996] References: PMID:9786946 Sources: GOC:dph, GOC:jl, GOC:mah, GOC:sgd_curators